{
  "gene_symbol": "TMEM278",
  "term_id": "GO:0090090",
  "gene": "UniProtKB:A6NKF7",
  "gene_name": "Transmembrane protein 88B",
  "term_label": "negative regulation of canonical Wnt signaling pathway"
}